{
  "term_id": "GO:0005665",
  "term_label": "RNA polymerase II, core complex",
  "gene_name": "DNA-directed RNA polymerases I, II, and III subunit RPABC5",
  "gene": "UniProtKB:P62875",
  "gene_symbol": "POLR2L"
}